{
  "term_id": "GO:0140767",
  "gene": "UniProtKB:P79522",
  "gene_name": "Proline-rich protein 3",
  "term_label": "enzyme-substrate adaptor activity",
  "gene_symbol": "PRR3"
}